{
  "gene_symbol": "PAQR8",
  "gene": "UniProtKB:Q8TEZ7",
  "term_label": "plasma membrane",
  "term_id": "GO:0005886",
  "gene_name": "Membrane progestin receptor beta"
}